Renilla-luciferin 2-monooxygenase activity [GO:0050248] (molecular function) Sources: EC:1.13.12.5, MetaCyc:RENILLA-LUCIFERIN-2-MONOOXYGENASE-RXN Definition: Catalysis of the reaction: Renilla luciferin + O2 = oxidized Renilla luciferin + CO2 + light. Relationships: is a type of oxidoreductase activity, acting on single donors with incorporation of molecular oxygen, incorporation of one atom of oxygen (internal monooxygenases or internal mixed function oxidases) [GO:0016703]; is a type of luciferin monooxygenase activity [GO:0045289] Also known as: luciferase activity, aequorin activity, Renilla-luciferin:oxygen 2-oxidoreductase (decarboxylating), Renilla-type luciferase activity, luciferase (Renilla luciferin)